{
  "gene_name": "Zinc finger protein 853",
  "term_id": "UNKNOWN:0003",
  "term_label": "Unknown cellular component",
  "gene": "UniProtKB:P0CG23",
  "gene_symbol": "ZNF853"
}